secondary branching, open tracheal system [GO:0007429] (biological process) Also known as: secondary tracheal branching References: PMID:29844090 Sources: GOC:mtg_sensu Definition: Sprouting of secondary branches in an open tracheal system. These form from the tips of primary branches and are formed by individual cells that roll up into unicellular tubes. An example of this is found in Drosophila melanogaster. Relationships: is a type of branching involved in open tracheal system development [GO:0060446]